tubulin deacetylase activity [GO:0042903] (molecular function) Relationships: is a type of hydrolase activity, acting on carbon-nitrogen (but not peptide) bonds, in linear amides [GO:0016811]; is a type of protein lysine deacetylase activity [GO:0033558] References: PMID:12024216, PMID:12486003 Definition: Catalysis of the reaction: N-acetyl(alpha-tubulin) + H2O = alpha-tubulin + acetate.